{
  "gene_name": "Microprocessor complex subunit DGCR8",
  "term_label": "double-stranded RNA binding",
  "term_id": "GO:0003725",
  "gene_symbol": "DGCR8",
  "gene": "UniProtKB:Q8WYQ5"
}